{
  "gene_name": "Uncharacterized protein C21orf62",
  "gene_symbol": "C21orf62",
  "term_label": "migrasome",
  "gene": "UniProtKB:Q9NYP8",
  "term_id": "GO:0140494"
}